imaginal disc-derived wing margin morphogenesis [GO:0008587] (biological process) Definition: The process in which the anatomical structures of the imaginal disc-derived wing margin are generated and organized. The wing margin is a strip of cells in the third instar disc at the boundary between the presumptive dorsal and ventral surfaces of the wing blade. Note: See also the fly_anatomy.ontology term 'wing margin ; FBbt:00005378'. Relationships: is a type of GO:0009886; is part of imaginal disc-derived wing morphogenesis [GO:0007476] Also known as: wing margin morphogenesis Sources: GOC:bf, GOC:mtg_sensu, ISBN:0879694238